regulation of free ubiquitin chain polymerization [GO:1904542] (biological process) Note: An example of this is PARK2 in human (UniProt symbol O60260) in PMID:24660806 (inferred from mutant phenotype). Definition: Any process that modulates the frequency, rate or extent of free ubiquitin chain polymerization. Relationships: is a type of regulation of protein polymerization [GO:0032271]; regulates free ubiquitin chain polymerization [GO:0010994] References: PMID:24660806 Sources: GOC:PARL, GOC:TermGenie, GOC:pad, GO_REF:0000058 Subtypes: negative regulation of free ubiquitin chain polymerization [GO:1904543], positive regulation of free ubiquitin chain polymerization [GO:1904544]